{
  "gene": "UniProtKB:Q9UII6",
  "gene_symbol": "DUSP13B",
  "term_label": "cytoplasm",
  "gene_name": "Dual specificity protein phosphatase 13 isoform B",
  "term_id": "GO:0005737"
}